carboxylic acid metabolic process [GO:0019752] (biological process) Sources: ISBN:0198506732 Relationships: is a type of GO:0043436 Also known as: carboxylic acid metabolism Subtypes: sulfur amino acid metabolic process [GO:0000096], N-acetylneuraminate metabolic process [GO:0006054], asparagine metabolic process [GO:0006528], threonine metabolic process [GO:0006566], icosanoid metabolic process [GO:0006690], GO:0009072, branched-chain amino acid metabolic process [GO:0009081], homoserine metabolic process [GO:0009092], gibberellin metabolic process [GO:0009685], GO:0018872, phthalate metabolic process [GO:0018963], L-ascorbic acid metabolic process [GO:0019852], fructoselysine metabolic process [GO:0030393], oxylipin metabolic process [GO:0031407], monocarboxylic acid metabolic process [GO:0032787], saturated monocarboxylic acid metabolic process [GO:0032788], glucosinolate biosynthetic process from homomethionine [GO:0033506], glucosinolate biosynthetic process from phenylalanine [GO:0033507], carnosine metabolic process [GO:0035498], dicarboxylic acid metabolic process [GO:0043648], carboxylic acid biosynthetic process [GO:0046394], carboxylic acid catabolic process [GO:0046395], UDP-glucuronate metabolic process [GO:0046398], GO:0046502, mannosylglycerate metabolic process [GO:0051478], tricarboxylic acid metabolic process [GO:0072350], N-acetylmuramic acid metabolic process [GO:0097172], branched-chain alpha-keto acid decarboxylation to branched-chain acyl-CoA [GO:0120552], proteinogenic amino acid metabolic process [GO:0170039], non-proteinogenic amino acid metabolic process [GO:0170041], monodictyphenone metabolic process [GO:1900813], tatiopterin metabolic process [GO:1900869], cephalosporin C metabolic process [GO:1901266], alpha-amino acid metabolic process [GO:1901605], GO:1902056 Definition: The chemical reactions and pathways involving carboxylic acids, any organic acid containing one or more carboxyl (COOH) groups or anions (COO-).